{
  "term_label": "RNA polymerase II cis-regulatory region sequence-specific DNA binding",
  "gene_symbol": "SCRT2",
  "term_id": "GO:0000978",
  "gene_name": "Transcriptional repressor scratch 2",
  "gene": "UniProtKB:Q9NQ03"
}